negative regulation of synaptic transmission, GABAergic [GO:0032229] (biological process) Definition: Any process that stops, prevents, or reduces the frequency, rate or extent of GABAergic synaptic transmission, the process of communication from a neuron to another neuron across a synapse using the neurotransmitter gamma-aminobutyric acid (GABA). Also known as: down regulation of synaptic transmission, GABAergic, down-regulation of synaptic transmission, GABAergic, downregulation of synaptic transmission, GABAergic, inhibition of synaptic transmission, GABAergic Sources: GOC:mah Relationships: is a type of regulation of synaptic transmission, GABAergic [GO:0032228]; is a type of negative regulation of synaptic transmission [GO:0050805]; negatively regulates synaptic transmission, GABAergic [GO:0051932]